{
  "term_id": "UNKNOWN:0002",
  "gene_name": "Zinc finger C2HC domain-containing protein 1B",
  "term_label": "Unknown biological process",
  "gene_symbol": "ZC2HC1B",
  "gene": "UniProtKB:Q5TFG8"
}